{
  "term_label": "scaffold protein binding",
  "gene_symbol": "TCOF1",
  "gene_name": "Treacle protein",
  "term_id": "GO:0097110",
  "gene": "UniProtKB:Q13428"
}